methionine racemase activity [GO:0018111] (molecular function) Sources: EC:5.1.1.2, RHEA:12492 Definition: Catalysis of the reaction: L-methionine = D-methionine. Relationships: is a type of GO:0047661